{
  "gene": "UniProtKB:Q9NVD7",
  "gene_name": "Alpha-parvin",
  "term_id": "GO:0005925",
  "gene_symbol": "PARVA",
  "term_label": "focal adhesion"
}